response to ketamine [GO:1901986] (biological process) Definition: Any process that results in a change in state or activity of a cell or an organism (in terms of movement, secretion, enzyme production, gene expression, etc.) as a result of a ketamine stimulus. Relationships: is_a response to ketone [GO:1901654]; is_a response to nitrogen compound [GO:1901698] References: PMID:11251190 Sources: GOC:TermGenie